{
  "term_id": "UNKNOWN:0001",
  "gene": "UniProtKB:Q9H2Y9",
  "term_label": "Unknown molecular function",
  "gene_name": "Solute carrier organic anion transporter family member 5A1",
  "gene_symbol": "SLCO5A1"
}